2,3-diketo-5-methylthiopentyl-1-phosphate enolase activity [GO:0043715] (molecular function) Note: This function is part of the process of methionine salvage. Definition: Catalysis of the reaction: 2,3-diketo-5-methylthiopentyl-1-phosphate = H+ + 2-hydroxy 3-keto-5-methylthiopentenyl-1-phosphate. 2,3-diketo-5-methylthiopentyl-1-phosphate is also known as DK-MTP-1-P, and 2-hydroxy 3-keto-5-methylthiopentenyl-1-phosphate as HK-MTPenyl-1-P. Sources: MetaCyc:R82-RXN Relationships: is a type of intramolecular oxidoreductase activity, interconverting keto- and enol-groups [GO:0016862] Also known as: DK-MTP-1-P enolase activity, E-1, MasA, mtnW